{
  "gene": "UniProtKB:Q9H871",
  "term_id": "GO:0005737",
  "gene_symbol": "RMND5A",
  "term_label": "cytoplasm",
  "gene_name": "E3 ubiquitin-protein transferase RMND5A"
}